positive regulation of tatiopterin biosynthetic process [GO:1900976] (biological process) Definition: Any process that activates or increases the frequency, rate or extent of tatiopterin biosynthetic process. Sources: GOC:TermGenie, GOC:mengo_curators Relationships: is a type of GO:0009891; is a type of GO:0010562; is_a positive regulation of small molecule metabolic process [GO:0062013]; is a type of regulation of tatiopterin biosynthetic process [GO:1900974]; positively regulates tatiopterin biosynthetic process [GO:1900870] Also known as: activation of tatiopterin anabolism, activation of tatiopterin biosynthesis, activation of tatiopterin formation, activation of tatiopterin synthesis, positive regulation of tatiopterin anabolism, positive regulation of tatiopterin biosynthesis, positive regulation of tatiopterin formation, positive regulation of tatiopterin synthesis, up regulation of tatiopterin anabolism, up regulation of tatiopterin biosynthesis, up regulation of tatiopterin biosynthetic process, up regulation of tatiopterin formation, up regulation of tatiopterin synthesis, up-regulation of tatiopterin anabolism, up-regulation of tatiopterin biosynthesis, up-regulation of tatiopterin biosynthetic process, up-regulation of tatiopterin formation, up-regulation of tatiopterin synthesis, upregulation of tatiopterin anabolism, upregulation of tatiopterin biosynthesis, upregulation of tatiopterin biosynthetic process, upregulation of tatiopterin formation, upregulation of tatiopterin synthesis, activation of tatiopterin biosynthetic process